{
  "gene": "UniProtKB:Q8TBK6",
  "term_id": "UNKNOWN:0001",
  "gene_name": "Zinc finger CCHC domain-containing protein 10",
  "gene_symbol": "ZCCHC10",
  "term_label": "Unknown molecular function"
}